{
  "gene_symbol": "DICER1",
  "term_id": "GO:0031054",
  "term_label": "pre-miRNA processing",
  "gene": "UniProtKB:Q9UPY3",
  "gene_name": "Endoribonuclease Dicer"
}